{
  "gene_name": "2-aminomuconic semialdehyde dehydrogenase",
  "gene": "UniProtKB:Q9H2A2",
  "gene_symbol": "ALDH8A1",
  "term_label": "retinal dehydrogenase (NAD+) activity",
  "term_id": "GO:0001758"
}